{
  "gene_name": "Protein patched homolog 2",
  "term_label": "hedgehog family protein binding",
  "term_id": "GO:0097108",
  "gene_symbol": "PTCH2",
  "gene": "UniProtKB:Q9Y6C5"
}